{
  "term_id": "GO:0000981",
  "term_label": "DNA-binding transcription factor activity, RNA polymerase II-specific",
  "gene": "UniProtKB:Q16559",
  "gene_name": "T-cell acute lymphocytic leukemia protein 2",
  "gene_symbol": "TAL2"
}